{
  "term_id": "GO:0005730",
  "gene_name": "rRNA 2'-O-methyltransferase fibrillarin",
  "term_label": "nucleolus",
  "gene": "UniProtKB:P22087",
  "gene_symbol": "FBL"
}